{
  "gene": "UniProtKB:P11487",
  "term_label": "fibroblast growth factor receptor signaling pathway",
  "term_id": "GO:0008543",
  "gene_name": "Fibroblast growth factor 3",
  "gene_symbol": "FGF3"
}